GDP-L-galactose biosynthetic process [GO:0033472] (biological process) Relationships: is a type of nucleotide-sugar biosynthetic process [GO:0009226] Also known as: GDP-L-galactose anabolism, GDP-L-galactose biosynthesis, GDP-L-galactose formation, GDP-L-galactose synthesis Sources: GOC:mah Definition: The chemical reactions and pathways resulting in the formation of GDP-L-galactose, a substance composed of L-galactose in glycosidic linkage with guanosine diphosphate.